{
  "term_id": "GO:0046332",
  "term_label": "SMAD binding",
  "gene": "UniProtKB:Q6ZNA4",
  "gene_name": "E3 ubiquitin-protein ligase Arkadia",
  "gene_symbol": "RNF111"
}